{
  "term_id": "UNKNOWN:0001",
  "gene_symbol": "LUZP2",
  "gene": "UniProtKB:Q86TE4",
  "term_label": "Unknown molecular function",
  "gene_name": "Leucine zipper protein 2"
}